inositol tetrakisphosphate kinase activity [GO:0051765] (molecular function) Subtypes: GO:0000824, inositol-1,3,4,5-tetrakisphosphate 6-kinase activity [GO:0000825], GO:0032942, inositol-3,4,5,6-tetrakisphosphate 1-kinase activity [GO:0047325], inositol-1,3,4,6-tetrakisphosphate 5-kinase activity [GO:0047326], inositol-1,3,4,6-tetrakisphosphate 2-kinase activity [GO:0102731] Relationships: is a type of phosphotransferase activity, alcohol group as acceptor [GO:0016773]; is a type of inositol phosphate kinase activity [GO:0180030] Sources: GOC:ai Definition: Catalysis of the reaction: inositol tetrakisphosphate + ATP = inositol pentakisphosphate + ADP.